{
  "gene_symbol": "CA1",
  "term_id": "GO:0005737",
  "gene": "UniProtKB:P00915",
  "gene_name": "Carbonic anhydrase 1",
  "term_label": "cytoplasm"
}